{
  "gene": "UniProtKB:Q96Q35",
  "term_id": "UNKNOWN:0002",
  "gene_symbol": "FLACC1",
  "gene_name": "Flagellum-associated coiled-coil domain-containing protein 1",
  "term_label": "Unknown biological process"
}